{
  "term_id": "GO:0016176",
  "gene_symbol": "SH3PXD2A",
  "term_label": "superoxide-generating NADPH oxidase activator activity",
  "gene": "UniProtKB:Q5TCZ1",
  "gene_name": "SH3 and PX domain-containing protein 2A"
}